{
  "gene_name": "Mimecan",
  "term_label": "bone development",
  "term_id": "GO:0060348",
  "gene_symbol": "OGN",
  "gene": "UniProtKB:P20774"
}